{
  "gene_name": "26S proteasome non-ATPase regulatory subunit 6",
  "gene": "UniProtKB:Q15008",
  "term_label": "proteasome-mediated ubiquitin-dependent protein catabolic process",
  "gene_symbol": "PSMD6",
  "term_id": "GO:0043161"
}